{
  "gene_symbol": "DMXL2",
  "gene": "UniProtKB:Q8TDJ6",
  "term_id": "GO:0007035",
  "term_label": "vacuolar acidification",
  "gene_name": "DmX-like protein 2"
}